{
  "term_id": "GO:0006959",
  "term_label": "humoral immune response",
  "gene_symbol": "IFNB1",
  "gene": "UniProtKB:P01574",
  "gene_name": "Interferon beta"
}